{
  "gene": "UniProtKB:Q9ULD2",
  "term_id": "GO:0005737",
  "gene_name": "Microtubule-associated tumor suppressor 1",
  "gene_symbol": "MTUS1",
  "term_label": "cytoplasm"
}